positive regulation of protein tetramerization [GO:1901092] (biological process) Relationships: is a type of positive regulation of protein oligomerization [GO:0032461]; is a type of regulation of protein tetramerization [GO:1901090]; positively regulates GO:0051262 Definition: Any process that activates or increases the frequency, rate or extent of protein tetramerization. Subtypes: GO:1901095 Sources: GOC:TermGenie, GOC:pm Also known as: positive regulation of protein tetramer assembly, positive regulation of protein tetramer biosynthesis, positive regulation of protein tetramer biosynthetic process, positive regulation of protein tetramer formation, up regulation of protein tetramer assembly, up regulation of protein tetramer biosynthesis, up regulation of protein tetramer biosynthetic process, up regulation of protein tetramer formation, up regulation of protein tetramerization, up-regulation of protein tetramer assembly, up-regulation of protein tetramer biosynthesis, up-regulation of protein tetramer biosynthetic process, up-regulation of protein tetramer formation, up-regulation of protein tetramerization, upregulation of protein tetramer assembly, upregulation of protein tetramer biosynthesis, upregulation of protein tetramer biosynthetic process, upregulation of protein tetramer formation, upregulation of protein tetramerization, activation of protein tetramer assembly, activation of protein tetramer biosynthesis, activation of protein tetramer biosynthetic process, activation of protein tetramer formation, activation of protein tetramerization